{
  "gene": "UniProtKB:O43464",
  "gene_name": "Serine protease HTRA2, mitochondrial",
  "gene_symbol": "HTRA2",
  "term_id": "GO:0006508",
  "term_label": "proteolysis"
}